{
  "term_label": "female pregnancy",
  "term_id": "GO:0007565",
  "gene": "UniProtKB:P15428",
  "gene_name": "15-hydroxyprostaglandin dehydrogenase [NAD(+)]",
  "gene_symbol": "HPGD"
}